{
  "gene": "UniProtKB:Q9BVA6",
  "gene_name": "Protein adenylyltransferase FICD",
  "term_label": "regulation of IRE1-mediated unfolded protein response",
  "gene_symbol": "FICD",
  "term_id": "GO:1903894"
}